{
  "term_id": "GO:0062030",
  "gene": "UniProtKB:Q9Y6J8",
  "gene_symbol": "STYXL1",
  "term_label": "negative regulation of stress granule assembly",
  "gene_name": "Serine_threonine_tyrosine-interacting-like protein 1"
}